oligosaccharide catabolic process [GO:0009313] (biological process) Definition: The chemical reactions and pathways resulting in the breakdown of oligosaccharides, molecules with between two and (about) 20 monosaccharide residues connected by glycosidic linkages. Sources: ISBN:0198506732 Relationships: is a type of oligosaccharide metabolic process [GO:0009311]; is a type of carbohydrate catabolic process [GO:0016052] Subtypes: raffinose catabolic process [GO:0034484], disaccharide catabolic process [GO:0046352], GO:0051681, cellodextrin catabolic process [GO:2000890], GO:2000894, cyclodextrin catabolic process [GO:2000901], GO:2000903, maltoheptaose catabolic process [GO:2001123] Also known as: oligosaccharide breakdown, oligosaccharide catabolism, oligosaccharide degradation, multicellular organismal oligosaccharide catabolic process